{
  "gene_symbol": "CRHR2",
  "gene": "UniProtKB:Q13324",
  "term_id": "GO:0007188",
  "term_label": "adenylate cyclase-modulating G protein-coupled receptor signaling pathway",
  "gene_name": "Corticotropin-releasing factor receptor 2"
}